{
  "gene_symbol": "NUP133",
  "term_id": "GO:0000972",
  "gene": "UniProtKB:Q8WUM0",
  "term_label": "transcription-dependent tethering of RNA polymerase II gene DNA at nuclear periphery",
  "gene_name": "Nuclear pore complex protein Nup133"
}